{
  "gene": "UniProtKB:Q96HZ7",
  "gene_name": "Putative uncharacterized protein URB1-AS1",
  "term_id": "UNKNOWN:0002",
  "term_label": "Unknown biological process",
  "gene_symbol": "URB1-AS1"
}